mitotic spindle organization [GO:0007052] (biological process) Definition: A process that is carried out at the cellular level which results in the assembly, arrangement of constituent parts, or disassembly of the microtubule spindle during a mitotic cell cycle. Regulation: regulated by regulation of mitotic spindle organization [GO:0060236]; positively regulated by positive regulation of mitotic spindle organization [GO:0110028] Note: In fission yeast most mitotic spindle organization occurs in the nucleus. Also known as: mitotic spindle organisation, spindle organization and biogenesis during mitosis, mitotic spindle organisation in nucleus, mitotic spindle organization and biogenesis in cell nucleus, mitotic spindle organization and biogenesis in nucleus, mitotic spindle organization in nucleus, spindle organization and biogenesis in nucleus during mitosis, mitotic spindle organization and biogenesis, mitotic spindle stabilization Relationships: is a type of spindle organization [GO:0007051]; is a type of GO:1902850 Subtypes: mitotic spindle disassembly [GO:0051228], mitotic spindle formation (spindle phase one) [GO:0061804], mitotic spindle elongation (spindle phase three) [GO:0061805], establishment of mitotic spindle asymmetry [GO:0061867], mitotic spindle assembly [GO:0090307] Sources: GOC:go_curators, GOC:mah